{
  "gene_name": "Transcription factor NF-E4",
  "gene": "UniProtKB:Q86UQ8",
  "term_id": "GO:0003712",
  "term_label": "transcription coregulator activity",
  "gene_symbol": "NFE4"
}